{
  "gene_name": "Immunoglobulin heavy variable 3-9",
  "term_label": "antigen binding",
  "gene": "UniProtKB:P01782",
  "term_id": "GO:0003823",
  "gene_symbol": "IGHV3-9"
}